{
  "gene_symbol": "TMED2",
  "gene": "UniProtKB:Q15363",
  "term_label": "intracellular protein transport",
  "gene_name": "Transmembrane emp24 domain-containing protein 2",
  "term_id": "GO:0006886"
}